{
  "term_label": "zymogen activation",
  "gene_symbol": "HGFAC",
  "term_id": "GO:0031638",
  "gene_name": "Hepatocyte growth factor activator",
  "gene": "UniProtKB:Q04756"
}